{
  "gene_symbol": "LEFTY2",
  "term_label": "BMP signaling pathway",
  "gene_name": "Left-right determination factor 2",
  "gene": "UniProtKB:O00292",
  "term_id": "GO:0030509"
}